{
  "term_label": "negative regulation of Golgi to plasma membrane protein transport",
  "gene_name": "Lysophospholipase-like protein 1",
  "gene": "UniProtKB:Q5VWZ2",
  "term_id": "GO:0042997",
  "gene_symbol": "LYPLAL1"
}